{
  "gene": "UniProtKB:A0A0G2JMH3",
  "gene_name": "ADP-ribosylation factor-like protein 17 C-terminal domain-containing protein",
  "term_label": "intracellular protein transport",
  "gene_symbol": "LOC107984156",
  "term_id": "GO:0006886"
}